{
  "gene_symbol": "KCNMB2",
  "gene_name": "Calcium-activated potassium channel subunit beta-2",
  "term_id": "GO:0015459",
  "term_label": "potassium channel regulator activity",
  "gene": "UniProtKB:Q9Y691"
}